{
  "gene": "UniProtKB:Q969M3",
  "term_label": "vesicle fusion with Golgi apparatus",
  "gene_symbol": "YIPF5",
  "gene_name": "Protein YIPF5",
  "term_id": "GO:0048280"
}